phosphatidylcholine flippase activity [GO:0140345] (molecular function) Definition: Catalysis of the movement of phosphatidylcholine from the exoplasmic to the cytosolic leaflet of a membrane, using energy from the hydrolysis of ATP. References: PMID:11870854 Also known as: phosphatidylcholine flippase activity (exoplasmic to cytosolic leaflet) Relationships: is a type of GO:0008525; is a type of glycerophospholipid flippase activity [GO:0140333]